{
  "gene_symbol": "Q8N9P0",
  "term_label": "Unknown cellular component",
  "gene": "UniProtKB:Q8N9P0",
  "gene_name": "Putative uncharacterized protein FLJ36797",
  "term_id": "UNKNOWN:0003"
}